alpha-adrenergic receptor activity [GO:0004936] (molecular function) Sources: GOC:mah, IUPHAR_GPCR:1274 Subtypes: GO:0004937, GO:0004938 Relationships: is a type of adrenergic receptor activity [GO:0004935] Also known as: alpha adrenoceptor Definition: Combining with epinephrine or norepinephrine to initiate a change in cell activity via activation of a G protein, with pharmacological characteristics of alpha-adrenergic receptors.